{
  "gene_name": "Prickle-like protein 2",
  "gene_symbol": "PRICKLE2",
  "term_label": "Unknown biological process",
  "term_id": "UNKNOWN:0002",
  "gene": "UniProtKB:Q7Z3G6"
}